{
  "gene_symbol": "NREP",
  "gene_name": "Neuronal regeneration-related protein",
  "gene": "UniProtKB:Q16612",
  "term_label": "regulation of neuron differentiation",
  "term_id": "GO:0045664"
}